flavone apiosyltransferase activity [GO:0047892] (molecular function) Also known as: UDP-apiose:5,4'-dihydroxyflavone 7-O-beta-D-glucoside 2''-O-beta-D-apiofuranosyltransferase activity, UDP-apiose:7-O-(beta-D-glucosyl)-flavone apiosyltransferase activity, uridine diphosphoapiose-flavone apiosyltransferase activity Definition: Catalysis of the reaction: UDP-apiose + 7-O-beta-D-glucosyl-5,7,4'-trihydroxyflavone = UDP + 7-O-(beta-D-apiofuranosyl-1,2-beta-D-glucosyl)-5,7,4'-trihydroxyflavone. Sources: EC:2.4.2.25, MetaCyc:FLAVONE-APIOSYLTRANSFERASE-RXN Relationships: is a type of UDP-glycosyltransferase activity [GO:0008194]; is a type of pentosyltransferase activity [GO:0016763]